{
  "term_label": "Cul7-RING ubiquitin ligase complex",
  "gene_name": "Cullin-9",
  "gene_symbol": "CUL9",
  "gene": "UniProtKB:Q8IWT3",
  "term_id": "GO:0031467"
}